presynaptic grid [GO:1990013] (cellular component) Sources: ISBN:0716723808, NIF_Subcellular:sao1730664005 Relationships: is a type of GO:0110165; is part of GO:0048786 Definition: A hexagonal array of electron dense particles attached to the cytoplasmic face of the presynaptic membrane. Also known as: pre-synaptic grid